{
  "term_label": "chromatin remodeling",
  "gene_symbol": "HDGFL1",
  "term_id": "GO:0006338",
  "gene": "UniProtKB:Q5TGJ6",
  "gene_name": "Hepatoma-derived growth factor-like protein 1"
}